norepinephrine biosynthetic process [GO:0042421] (biological process) Sources: GOC:jl, ISBN:0198506732 Definition: The chemical reactions and pathways resulting in the formation of norepinephrine, a hormone secreted by the adrenal medulla, and a neurotransmitter in the sympathetic peripheral nervous system and in some tracts in the central nervous system. It is also the demethylated biosynthetic precursor of epinephrine. Relationships: is a type of GO:0042415; is_a catecholamine biosynthetic process [GO:0042423] Also known as: levarterenol biosynthesis, levarterenol biosynthetic process, noradrenaline biosynthesis, noradrenaline biosynthetic process, norepinephrine anabolism, norepinephrine biosynthesis, norepinephrine formation, norepinephrine synthesis